negative regulation of establishment of Sertoli cell barrier [GO:1904445] (biological process) Definition: Any process that stops, prevents or reduces the frequency, rate or extent of establishment of Sertoli cell barrier. Also known as: down regulation of establishment of BTB, down regulation of establishment of SCB, down regulation of establishment of Sertoli cell barrier, down regulation of establishment of blood-testis barrier, down-regulation of establishment of BTB, down-regulation of establishment of SCB, down-regulation of establishment of Sertoli cell barrier, down-regulation of establishment of blood-testis barrier, downregulation of establishment of BTB, downregulation of establishment of SCB, downregulation of establishment of Sertoli cell barrier, downregulation of establishment of blood-testis barrier, negative regulation of establishment of BTB, negative regulation of establishment of SCB, negative regulation of establishment of blood-testis barrier, inhibition of establishment of BTB, inhibition of establishment of SCB, inhibition of establishment of Sertoli cell barrier, inhibition of establishment of blood-testis barrier Relationships: is a type of negative regulation of cell development [GO:0010721]; is a type of GO:0030857; is a type of regulation of establishment of Sertoli cell barrier [GO:1904444]; is a type of negative regulation of reproductive process [GO:2000242]; negatively regulates GO:0097368 References: PMID:18057314 Sources: GOC:TermGenie, GO_REF:0000058